{
  "term_id": "GO:0050968",
  "gene": "UniProtKB:O75762",
  "term_label": "detection of chemical stimulus involved in sensory perception of pain",
  "gene_name": "Transient receptor potential cation channel subfamily A member 1",
  "gene_symbol": "TRPA1"
}